{
  "gene_name": "T cell receptor beta variable 6-3",
  "gene_symbol": "TRBV6-3",
  "term_label": "plasma membrane",
  "term_id": "GO:0005886",
  "gene": "UniProtKB:P0DPF7"
}